{
  "gene": "UniProtKB:Q5W0Z9",
  "term_label": "synaptic vesicle maturation",
  "gene_symbol": "ZDHHC20",
  "term_id": "GO:0016188",
  "gene_name": "Palmitoyltransferase ZDHHC20"
}